{
  "gene": "UniProtKB:O15550",
  "gene_name": "Lysine-specific demethylase 6A",
  "gene_symbol": "KDM6A",
  "term_id": "GO:0000978",
  "term_label": "RNA polymerase II cis-regulatory region sequence-specific DNA binding"
}